negative regulation of reverse transcription [GO:1900269] (biological process) Also known as: down regulation of reverse transcription, down-regulation of reverse transcription, downregulation of reverse transcription, inhibition of reverse transcription Sources: GOC:TermGenie Relationships: is a type of regulation of reverse transcription [GO:1900268]; is a type of negative regulation of DNA biosynthetic process [GO:2000279]; negatively regulates reverse transcription [GO:0001171] Definition: Any process that stops, prevents or reduces the frequency, rate or extent of reverse transcription.